naringenin-chalcone synthase activity [GO:0016210] (molecular function) Definition: Catalysis of the reaction: 3 malonyl-CoA + 4-coumaroyl-CoA = 4 CoA + naringenin chalcone + 3 CO2. Sources: EC:2.3.1.74 Also known as: malonyl-CoA:4-coumaroyl-CoA malonyltransferase (cyclizing), DOCS Relationships: is a type of acyltransferase activity, transferring groups other than amino-acyl groups [GO:0016747]